platelet alpha granule organization [GO:0070889] (biological process) References: PMID:16123220 Sources: GOC:rph Definition: A process that is carried out at the cellular level which results in the assembly, arrangement of constituent parts, or disassembly of a platelet alpha granule. A platelet alpha granule is a secretory organelle found in blood platelets. Relationships: is_a secretory granule organization [GO:0033363] Also known as: platelet alpha granule organisation, platelet alpha-granule organization, platelet alpha granule organization and biogenesis